{
  "term_id": "GO:0042832",
  "gene": "UniProtKB:Q96PP9",
  "gene_name": "Guanylate-binding protein 4",
  "gene_symbol": "GBP4",
  "term_label": "defense response to protozoan"
}